{
  "gene_name": "Kinetochore protein Nuf2",
  "gene_symbol": "NUF2",
  "gene": "UniProtKB:Q9BZD4",
  "term_label": "mitotic spindle organization",
  "term_id": "GO:0007052"
}